{
  "term_id": "GO:0005737",
  "gene": "UniProtKB:Q96H55",
  "gene_symbol": "MYO19",
  "gene_name": "Unconventional myosin-XIX",
  "term_label": "cytoplasm"
}